{
  "gene": "UniProtKB:Q8NG11",
  "gene_name": "Tetraspanin-14",
  "term_label": "Unknown biological process",
  "term_id": "UNKNOWN:0002",
  "gene_symbol": "TSPAN14"
}